{
  "term_label": "Unknown biological process",
  "term_id": "UNKNOWN:0002",
  "gene": "UniProtKB:Q9H2C8",
  "gene_name": "Olfactory receptor 51V1",
  "gene_symbol": "OR51V1"
}